negative regulation of RNA polymerase II transcription preinitiation complex assembly [GO:0017055] (biological process) Definition: Any process that stops, prevents, or reduces the frequency, rate or extent of RNA polymerase II transcriptional preinitiation complex assembly. Also known as: down regulation of RNA polymerase II transcriptional preinitiation complex assembly, down-regulation of RNA polymerase II transcriptional preinitiation complex assembly, downregulation of RNA polymerase II transcriptional preinitiation complex assembly, negative regulation of RNA polymerase II transcriptional pre-initiation complex assembly, negative regulation of RNA polymerase II transcriptional pre-initiation complex biosynthesis, negative regulation of RNA polymerase II transcriptional preinitiation complex assembly, negative regulation of RNA polymerase II transcriptional preinitiation complex formation, inhibition of RNA polymerase II transcriptional preinitiation complex assembly Relationships: is a type of negative regulation of protein-containing complex assembly [GO:0031333]; is a type of regulation of RNA polymerase II transcription preinitiation complex assembly [GO:0045898]; is a type of negative regulation of transcription initiation by RNA polymerase II [GO:0060633]; negatively regulates RNA polymerase II preinitiation complex assembly [GO:0051123] Sources: GOC:go_curators